{
  "term_id": "UNKNOWN:0002",
  "gene_symbol": "ZNRD2",
  "gene": "UniProtKB:O60232",
  "term_label": "Unknown biological process",
  "gene_name": "Protein ZNRD2"
}